{
  "gene": "UniProtKB:Q96BT7",
  "term_id": "GO:0005634",
  "gene_symbol": "ALKBH8",
  "term_label": "nucleus",
  "gene_name": "Alkylated DNA repair protein alkB homolog 8"
}